{
  "gene_symbol": "ODF4",
  "term_id": "UNKNOWN:0002",
  "gene_name": "Outer dense fiber protein 4",
  "term_label": "Unknown biological process",
  "gene": "UniProtKB:Q2M2E3"
}